{
  "gene_name": "3-mercaptopyruvate sulfurtransferase",
  "term_label": "tRNA wobble position uridine thiolation",
  "term_id": "GO:0002143",
  "gene_symbol": "MPST",
  "gene": "UniProtKB:P25325"
}